cellular response to biphenyl [GO:1904615] (biological process) Definition: Any process that results in a change in state or activity of a cell (in terms of movement, secretion, enzyme production, gene expression, etc.) as a result of a biphenyl stimulus. References: PMID:23196670 Sources: GOC:TermGenie, GO_REF:0000071 Relationships: is a type of cellular response to chemical stimulus [GO:0070887]; is a type of response to biphenyl [GO:1904614]